syntaxin-3 binding [GO:0030348] (molecular function) Sources: GOC:ai Definition: Binding to a syntaxin-3 SNAP receptor. Relationships: is a type of GO:0019905